{
  "gene": "UniProtKB:Q00013",
  "term_label": "cell-cell junction",
  "gene_name": "55 kDa erythrocyte membrane protein",
  "gene_symbol": "MPP1",
  "term_id": "GO:0005911"
}